catalytic activity [GO:0003824] (molecular function) Sources: GOC:vw, ISBN:0198506732 Also known as: enzyme activity Subtypes: GO:0009975, polyketide synthase activity [GO:0016218], oxidoreductase activity [GO:0016491], transferase activity [GO:0016740], GO:0016787, GO:0016829, isomerase activity [GO:0016853], GO:0016874, demethylase activity [GO:0032451], GO:0061783, catalytic activity, acting on a protein [GO:0140096], catalytic activity, acting on a nucleic acid [GO:0140640], deacylase activity [GO:0160215], non-ribosomal peptide synthetase activity [GO:1904091] Regulation: negatively regulated by enzyme inhibitor activity [GO:0004857]; positively regulated by enzyme activator activity [GO:0008047]; regulated by enzyme regulator activity [GO:0030234]; positively regulated by positive regulation of catalytic activity [GO:0043085]; negatively regulated by negative regulation of catalytic activity [GO:0043086]; regulated by modulation by host of viral catalytic activity [GO:0044867]; regulated by regulation of catalytic activity [GO:0050790] Relationships: is a type of molecular_function [GO:0003674] Definition: Catalysis of a biochemical reaction at physiological temperatures. In biologically catalyzed reactions, the reactants are known as substrates, and the catalysts are naturally occurring macromolecular substances known as enzymes. Enzymes possess specific binding sites for substrates, and are usually composed wholly or largely of protein, but RNA that has catalytic activity (ribozyme) is often also regarded as enzymatic.